negative regulation of adult salivary gland boundary specification [GO:0045709] (biological process) Definition: Any process that stops, prevents, or reduces the frequency, rate or extent of salivary gland determination in an adult organism. Sources: GOC:go_curators, GOC:tb Also known as: down regulation of adult salivary gland determination, down-regulation of adult salivary gland determination, downregulation of adult salivary gland determination, negative regulation of adult salivary gland determination, inhibition of adult salivary gland determination Relationships: is a type of GO:0045705; is a type of regulation of adult salivary gland boundary specification [GO:0045707]; negatively regulates adult salivary gland boundary specification [GO:0007434]